beta-1,2-oligomannoside biosynthetic process [GO:0070136] (biological process) References: PMID:18234669 Sources: GOC:mah Also known as: beta-1,2-oligomannoside anabolism, beta-1,2-oligomannoside biosynthesis, beta-1,2-oligomannoside formation, beta-1,2-oligomannoside synthesis Relationships: is a type of GO:0046354; is a type of fungal-type cell wall polysaccharide biosynthetic process [GO:0051278]; is a type of beta-1,2-oligomannoside metabolic process [GO:0070135] Definition: The chemical reactions and pathways resulting in the formation of beta-1,2-linked oligomannosides, which are found in fungal cell wall phosphopeptidomannan and phospholipomannan.